{
  "term_label": "transcription corepressor binding",
  "gene": "UniProtKB:P56645",
  "gene_name": "Period circadian protein homolog 3",
  "term_id": "GO:0001222",
  "gene_symbol": "PER3"
}